{
  "gene_name": "Activin receptor type-1",
  "gene_symbol": "ACVR1",
  "gene": "UniProtKB:Q04771",
  "term_label": "dorsal/ventral pattern formation",
  "term_id": "GO:0009953"
}